protein targeting to vacuolar membrane [GO:0044395] (BP) Relationships: is a type of protein targeting to membrane [GO:0006612]; is a type of protein targeting to vacuole [GO:0006623]; is a type of protein localization to vacuolar membrane [GO:1903778] Regulation: regulated by regulation of protein targeting to vacuolar membrane [GO:1900483]; negatively regulated by negative regulation of protein targeting to vacuolar membrane [GO:1900484]; positively regulated by positive regulation of protein targeting to vacuolar membrane [GO:1900485] Sources: GOC:jl Definition: The process of directing proteins towards the vacuolar membrane; usually uses signals contained within the protein.